{
  "term_label": "neutral L-amino acid transmembrane transporter activity",
  "gene": "UniProtKB:P43003",
  "gene_name": "Excitatory amino acid transporter 1",
  "gene_symbol": "SLC1A3",
  "term_id": "GO:0015175"
}